{
  "gene_symbol": "RXFP2",
  "gene": "UniProtKB:Q8WXD0",
  "gene_name": "Relaxin receptor 2",
  "term_id": "GO:0005886",
  "term_label": "plasma membrane"
}